{
  "term_id": "GO:0005096",
  "gene_name": "TBC1 domain family member 25",
  "gene_symbol": "TBC1D25",
  "gene": "UniProtKB:Q3MII6",
  "term_label": "GTPase activator activity"
}